{
  "gene": "UniProtKB:Q96HM7",
  "gene_name": "PC-esterase domain-containing protein 1B",
  "gene_symbol": "PCED1B",
  "term_id": "UNKNOWN:0001",
  "term_label": "Unknown molecular function"
}